{
  "term_id": "GO:0038131",
  "term_label": "neuregulin receptor activity",
  "gene_name": "Receptor tyrosine-protein kinase erbB-3",
  "gene_symbol": "ERBB3",
  "gene": "UniProtKB:P21860"
}